{
  "term_id": "GO:0008379",
  "term_label": "thioredoxin peroxidase activity",
  "gene_name": "Peroxiredoxin-5, mitochondrial",
  "gene_symbol": "PRDX5",
  "gene": "UniProtKB:P30044"
}